{
  "term_label": "cell projection membrane",
  "term_id": "GO:0031253",
  "gene": "UniProtKB:Q9NQT6",
  "gene_symbol": "FSCN3",
  "gene_name": "Fascin-3"
}